{
  "gene": "UniProtKB:Q96FE7",
  "term_label": "signaling receptor binding",
  "gene_symbol": "PIK3IP1",
  "term_id": "GO:0005102",
  "gene_name": "Phosphoinositide-3-kinase-interacting protein 1"
}